{
  "term_id": "UNKNOWN:0002",
  "gene": "UniProtKB:Q5TA79",
  "gene_symbol": "LCE2A",
  "term_label": "Unknown biological process",
  "gene_name": "Late cornified envelope protein 2A"
}